follicle cell of egg chamber stalk formation [GO:0030713] (biological process) Relationships: is a type of cell morphogenesis [GO:0000902]; is a type of developmental process involved in reproduction [GO:0003006]; is part of follicle cell of egg chamber development [GO:0030707] Definition: Development of ovarian follicle cells to create the interfollicular stalks that connect the egg chambers of progressive developmental stages. An example of this process is found in Drosophila melanogaster. References: PMID:10822261 Sources: GOC:mtg_sensu